{
  "term_id": "GO:0017148",
  "gene_name": "Nanos homolog 1",
  "gene": "UniProtKB:Q8WY41",
  "gene_symbol": "NANOS1",
  "term_label": "negative regulation of translation"
}